{
  "term_label": "Unknown molecular function",
  "gene_symbol": "C1orf162",
  "gene": "UniProtKB:Q8NEQ5",
  "gene_name": "Transmembrane protein C1orf162",
  "term_id": "UNKNOWN:0001"
}